{
  "gene": "UniProtKB:O76038",
  "gene_name": "Secretagogin",
  "gene_symbol": "SCGN",
  "term_id": "GO:0005509",
  "term_label": "calcium ion binding"
}